regulation of transcription regulatory region DNA binding [GO:2000677] (biological process) Definition: Any process that modulates the frequency, rate or extent of transcription regulatory region DNA binding. Relationships: is a type of regulation of DNA binding [GO:0051101]; regulates GO:0000976 Sources: GOC:obol Subtypes: regulation of RNA polymerase II regulatory region sequence-specific DNA binding [GO:1903025], negative regulation of transcription regulatory region DNA binding [GO:2000678], positive regulation of transcription regulatory region DNA binding [GO:2000679]